{
  "gene_name": "KN motif and ankyrin repeat domain-containing protein 1",
  "gene_symbol": "KANK1",
  "gene": "UniProtKB:Q14678",
  "term_label": "cytoplasm",
  "term_id": "GO:0005737"
}